{
  "gene_symbol": "VPS25",
  "gene_name": "Vacuolar protein-sorting-associated protein 25",
  "gene": "UniProtKB:Q9BRG1",
  "term_id": "GO:0042803",
  "term_label": "protein homodimerization activity"
}